{
  "term_label": "maturation of SSU-rRNA from tricistronic rRNA transcript (SSU-rRNA, 5.8S rRNA, LSU-rRNA)",
  "term_id": "GO:0000462",
  "gene_name": "Pre-rRNA-processing protein TSR1 homolog",
  "gene_symbol": "TSR1",
  "gene": "UniProtKB:Q2NL82"
}